{
  "term_id": "UNKNOWN:0001",
  "term_label": "Unknown molecular function",
  "gene": "UniProtKB:Q13087",
  "gene_name": "Protein disulfide-isomerase A2",
  "gene_symbol": "PDIA2"
}